{
  "gene_name": "Cofilin-1",
  "gene": "UniProtKB:P23528",
  "gene_symbol": "CFL1",
  "term_id": "GO:0030027",
  "term_label": "lamellipodium"
}